{
  "gene": "UniProtKB:Q01538",
  "gene_name": "Myelin transcription factor 1",
  "term_label": "Unknown molecular function",
  "term_id": "UNKNOWN:0001",
  "gene_symbol": "MYT1"
}